{
  "term_id": "GO:0005737",
  "gene_symbol": "TRIM58",
  "term_label": "cytoplasm",
  "gene_name": "E3 ubiquitin-protein ligase TRIM58",
  "gene": "UniProtKB:Q8NG06"
}